pyrazolylalanine synthase activity [GO:0050234] (molecular function) Sources: EC:4.2.1.50, RHEA:24512 Definition: Catalysis of the reaction: L-serine + pyrazole = 3-(pyrazol-1-yl)-L-alanine + H2O. Relationships: is a type of hydro-lyase activity [GO:0016836] Also known as: L-serine hydro-lyase (adding pyrazole), L-serine hydro-lyase [adding pyrazole; 3-(pyrazol-1-yl)-L-alanine-forming], beta-pyrazolylalaninase activity